interleukin-35 binding [GO:0070746] (molecular function) Also known as: IL-35 binding Relationships: is a type of cytokine binding [GO:0019955] Sources: GOC:add Definition: Binding to interleukin-35.